cellular response to tumor necrosis factor [GO:0071356] (biological process) Sources: GOC:mah Definition: Any process that results in a change in state or activity of a cell (in terms of movement, secretion, enzyme production, gene expression, etc.) as a result of a tumor necrosis factor stimulus. Relationships: is a type of GO:0034612; is a type of cellular response to cytokine stimulus [GO:0071345] Also known as: cellular response to TNF